{
  "term_id": "GO:0030187",
  "term_label": "melatonin biosynthetic process",
  "gene_symbol": "AANAT",
  "gene": "UniProtKB:Q16613",
  "gene_name": "Serotonin N-acetyltransferase"
}